{
  "term_label": "extracellular space",
  "gene": "UniProtKB:P00709",
  "gene_name": "Alpha-lactalbumin",
  "term_id": "GO:0005615",
  "gene_symbol": "LALBA"
}